{
  "gene_name": "3'-5' RNA helicase YTHDC2",
  "gene": "UniProtKB:Q9H6S0",
  "gene_symbol": "YTHDC2",
  "term_label": "Unknown biological process",
  "term_id": "UNKNOWN:0002"
}